{
  "term_label": "cytoplasm",
  "gene_symbol": "TUBB4A",
  "gene_name": "Tubulin beta-4A chain",
  "gene": "UniProtKB:P04350",
  "term_id": "GO:0005737"
}